nBAF complex [GO:0071565] (cellular component) References: PMID:17640523 Sources: GOC:mah, GOC:ss Relationships: is a type of SWI/SNF superfamily-type complex [GO:0070603] Definition: A SWI/SNF-type complex that is found in post-mitotic neurons, and in human contains actin and proteins encoded by the ARID1A/BAF250A or ARID1B/BAF250B, SMARCD1/BAF60A, SMARCD3/BAF60C, SMARCA2/BRM/BAF190B, SMARCA4/BRG1/BAF190A, SMARCB1/BAF47, SMARCC1/BAF155, SMARCE1/BAF57, SMARCC2/BAF170, DPF1/BAF45B, DPF3/BAF45C, ACTL6B/BAF53B genes. The nBAF complex along with CREST plays a role regulating the activity of genes essential for dendrite growth.